{
  "gene_name": "Galectin-3",
  "term_label": "immunological synapse",
  "gene_symbol": "LGALS3",
  "gene": "UniProtKB:P17931",
  "term_id": "GO:0001772"
}